{
  "gene": "UniProtKB:O15525",
  "gene_symbol": "MAFG",
  "term_label": "regulation of epidermal cell differentiation",
  "term_id": "GO:0045604",
  "gene_name": "Transcription factor MafG"
}